{
  "gene": "UniProtKB:Q8TB52",
  "term_id": "UNKNOWN:0002",
  "term_label": "Unknown biological process",
  "gene_name": "F-box only protein 30",
  "gene_symbol": "FBXO30"
}